{
  "term_label": "Unknown biological process",
  "gene_name": "STAGA complex 65 subunit gamma",
  "gene_symbol": "SUPT7L",
  "gene": "UniProtKB:O94864",
  "term_id": "UNKNOWN:0002"
}